{
  "gene_symbol": "POLD4",
  "term_label": "DNA-templated DNA replication",
  "gene_name": "DNA polymerase delta subunit 4",
  "term_id": "GO:0006261",
  "gene": "UniProtKB:Q9HCU8"
}